{
  "term_label": "sensory perception of smell",
  "gene_symbol": "SLC24A4",
  "term_id": "GO:0007608",
  "gene": "UniProtKB:Q8NFF2",
  "gene_name": "Sodium_potassium_calcium exchanger 4"
}